negative regulation of mineralocorticoid secretion [GO:2000856] (biological process) Relationships: is_a negative regulation of corticosteroid hormone secretion [GO:2000847]; is a type of GO:2000855; negatively regulates mineralocorticoid secretion [GO:0035931] Subtypes: negative regulation of aldosterone secretion [GO:2000859] Sources: GOC:sl Definition: Any process that stops, prevents or reduces the frequency, rate or extent of mineralocorticoid secretion.